{
  "term_id": "GO:0005794",
  "gene_symbol": "ZFPL1",
  "gene": "UniProtKB:O95159",
  "gene_name": "Zinc finger protein-like 1",
  "term_label": "Golgi apparatus"
}